palmitoyl-CoA ligase activity [GO:0090433] (molecular function) Definition: Catalysis of the reaction: ATP + palmitic acid + CoA = AMP + diphosphate + palmitoyl-CoA. Also known as: palmitoyl-CoA synthetase activity Relationships: is a type of long-chain fatty acid-CoA ligase activity [GO:0004467] References: PMID:18071249 Sources: GOC:al